amyloid-beta clearance [GO:0097242] (biological process) Relationships: is_a multicellular organismal process [GO:0032501] Definition: The process in which amyloid-beta is removed from extracellular brain regions by mechanisms involving cell surface receptors. References: PMID:18289866, PMID:19098903, PMID:26005850 Sources: GOC:BHF, GOC:aruk, GOC:bc Regulation: RO_0002211 by regulation of amyloid-beta clearance [GO:1900221]; RO_0002212 by negative regulation of amyloid-beta clearance [GO:1900222]; positively regulated by positive regulation of amyloid-beta clearance [GO:1900223] Also known as: beta-amyloid clearance Subtypes: amyloid-beta clearance by transcytosis [GO:0150093], amyloid-beta clearance by cellular catabolic process [GO:0150094]